{
  "gene": "UniProtKB:P50552",
  "gene_name": "Vasodilator-stimulated phosphoprotein",
  "term_label": "axon guidance",
  "term_id": "GO:0007411",
  "gene_symbol": "VASP"
}